{
  "term_label": "Unknown biological process",
  "term_id": "UNKNOWN:0002",
  "gene_name": "Uncharacterized protein",
  "gene_symbol": "A0A804HJT0",
  "gene": "UniProtKB:A0A804HJT0"
}